cuticle hydrocarbon biosynthetic process [GO:0006723] (biological process) Relationships: is a type of hydrocarbon biosynthetic process [GO:0120251]; is part of GO:0042335 Sources: GOC:ai Definition: The chemical reactions and pathways resulting in the formation of hydrocarbons that make up the cuticle, the outer layer of some animals and plants, which acts to prevent water loss. Also known as: cuticle hydrocarbon anabolism, cuticle hydrocarbon biosynthesis, cuticle hydrocarbon formation, cuticle hydrocarbon synthesis